non-membrane spanning protein tyrosine phosphatase activity [GO:0004726] (molecular function) References: PMID:34353440 Relationships: is a type of GO:0004725 Definition: Catalysis of the reaction: non-membrane spanning protein tyrosine phosphate + H2O = non-membrane spanning protein tyrosine + phosphate.